{
  "gene_symbol": "CCND2",
  "gene": "UniProtKB:P30279",
  "term_label": "cytoplasm",
  "gene_name": "G1_S-specific cyclin-D2",
  "term_id": "GO:0005737"
}